{
  "gene": "UniProtKB:Q29983",
  "term_label": "gamma-delta T cell activation",
  "gene_name": "MHC class I polypeptide-related sequence A",
  "gene_symbol": "MICA",
  "term_id": "GO:0046629"
}